{
  "term_id": "GO:0006355",
  "gene": "UniProtKB:Q6AWC2",
  "term_label": "regulation of DNA-templated transcription",
  "gene_symbol": "WWC2",
  "gene_name": "Protein WWC2"
}